synaptic vesicle docking [GO:0016081] (biological process) Definition: The initial (indirect) attachment of a synaptic vesicle membrane to the presynaptic active zone membrane, mediated by proteins protruding from the membrane and proteins of the presynaptic active zone cytoplasmic component. Synaptic vesicle tethering is the first step in this process. References: PMID:15217342 Also known as: synaptic vesicle docking involved in exocytosis, synaptic vesicle docking during exocytosis Note: Although this process can occur outside of synaptic transmission, by convention we treat it as a part of synaptic transmission (dos, pvn, fk synapse project 2015). Relationships: is a type of vesicle docking involved in exocytosis [GO:0006904]; is part of GO:0016079 Regulation: regulated by GO:0099148